{
  "gene": "UniProtKB:A2RRL7",
  "term_id": "UNKNOWN:0001",
  "gene_name": "Transmembrane protein 213",
  "gene_symbol": "TMEM213",
  "term_label": "Unknown molecular function"
}